{
  "gene_symbol": "GJD2",
  "term_id": "GO:0005922",
  "gene_name": "Gap junction delta-2 protein",
  "gene": "UniProtKB:Q9UKL4",
  "term_label": "connexin complex"
}